{
  "term_label": "external side of plasma membrane",
  "term_id": "GO:0009897",
  "gene": "UniProtKB:Q6UX52",
  "gene_name": "Protein IL-40",
  "gene_symbol": "C17orf99"
}